{
  "gene": "UniProtKB:Q8N957",
  "gene_name": "Ankyrin repeat and fibronectin type-III domain-containing protein 1",
  "term_id": "GO:0005819",
  "term_label": "spindle",
  "gene_symbol": "ANKFN1"
}